{
  "term_id": "GO:0000243",
  "gene_name": "Small nuclear ribonucleoprotein Sm D1",
  "term_label": "commitment complex",
  "gene": "UniProtKB:P62314",
  "gene_symbol": "SNRPD1"
}